{
  "gene": "UniProtKB:Q9H9H5",
  "gene_symbol": "MAP6D1",
  "term_label": "microtubule binding",
  "gene_name": "MAP6 domain-containing protein 1",
  "term_id": "GO:0008017"
}